aspartic-type endopeptidase activity [GO:0004190] (molecular function) Definition: Catalysis of the hydrolysis of internal, alpha-peptide bonds in a polypeptide chain by a mechanism in which a water molecule bound by the side chains of aspartic residues at the active center acts as a nucleophile. Relationships: is a type of endopeptidase activity [GO:0004175]; is_a aspartic-type peptidase activity [GO:0070001] Also known as: aspartic endopeptidase activity, aspartate protease activity, aspartic protease activity, aspartyl protease activity, carboxyl protease activity Sources: ISBN:0198506732 Subtypes: GO:0042500 Regulation: negatively regulated by aspartic-type endopeptidase inhibitor activity [GO:0019828]